aryl sulfotransferase activity [GO:0004062] (molecular function) Also known as: arylsulfotransferase, aryl sulphotransferase activity, 1-naphthol phenol sulfotransferase activity, 2-naphtholsulfotransferase activity, 3'-phosphoadenylyl-sulfate:phenol sulfotransferase activity, 4-nitrocatechol sulfokinase activity, PST, dopamine sulfotransferase activity, p-nitrophenol sulfotransferase activity, phenol sulfokinase activity, phenol sulfotransferase activity, ritodrine sulfotransferase activity, sulfokinase activity Relationships: is a type of GO:0008146 Definition: Catalysis of the reaction: 3'-phosphoadenosine 5'-phosphosulfate + a phenol = adenosine 3',5'-bisphosphate + an aryl sulfate. Sources: EC:2.8.2.1